regulation of membrane potential [GO:0042391] (biological process) Sources: GOC:jl, GOC:mtg_cardio, GOC:tb, ISBN:0198506732 Relationships: is a type of regulation of biological quality [GO:0065008]; has part monoatomic ion transmembrane transport [GO:0034220] Definition: Any process that modulates the establishment or extent of a membrane potential, the electric potential existing across any membrane arising from charges in the membrane itself and from the charges present in the media on either side of the membrane. Subtypes: action potential [GO:0001508], regulation of membrane depolarization [GO:0003254], regulation of membrane potential in photoreceptor cell [GO:0016057], stabilization of membrane potential [GO:0030322], negative regulation of membrane potential [GO:0045837], positive regulation of membrane potential [GO:0045838], regulation of mitochondrial membrane potential [GO:0051881], membrane depolarization [GO:0051899], regulation of resting membrane potential [GO:0060075], GO:0060078, membrane hyperpolarization [GO:0060081], regulation of membrane repolarization [GO:0060306], membrane repolarization [GO:0086009], GO:0086036, modulation of excitatory postsynaptic potential [GO:0098815], modulation of inhibitory postsynaptic potential [GO:0098828], spike train [GO:0098874], regulation of action potential [GO:0098900], regulation of presynaptic membrane potential [GO:0099505], regulation of membrane hyperpolarization [GO:1902630]